{
  "term_label": "Notch signaling pathway",
  "gene_symbol": "DLL1",
  "gene_name": "Delta-like protein 1",
  "gene": "UniProtKB:O00548",
  "term_id": "GO:0007219"
}